{
  "gene_name": "Protein arginine N-methyltransferase 7",
  "term_label": "protein-arginine N-methyltransferase activity",
  "gene": "UniProtKB:Q9NVM4",
  "gene_symbol": "PRMT7",
  "term_id": "GO:0016274"
}